{
  "gene": "UniProtKB:Q9UIW2",
  "gene_symbol": "PLXNA1",
  "term_id": "GO:0005886",
  "term_label": "plasma membrane",
  "gene_name": "Plexin-A1"
}